{
  "term_id": "GO:0001525",
  "gene_name": "Transcription factor SOX-18",
  "gene": "UniProtKB:P35713",
  "term_label": "angiogenesis",
  "gene_symbol": "SOX18"
}